{
  "gene_symbol": "ATXN3L",
  "gene": "UniProtKB:Q9H3M9",
  "term_id": "GO:0043161",
  "term_label": "proteasome-mediated ubiquitin-dependent protein catabolic process",
  "gene_name": "Ataxin-3-like protein"
}